lambda-carrageenase activity [GO:0033957] (molecular function) Definition: Catalysis of the endohydrolysis of beta-1,4-linkages in the backbone of lambda-carrageenan, resulting in the tetrasaccharide alpha-D-Galp2,6S2-(1->3)-beta-D-Galp2S-(1->4)-alpha-D-Galp2,6S2-(1->3)-D-Galp2S. Sources: EC:3.2.1.162 Also known as: endo-beta-1,4-carrageenose 2,6,2'-trisulfate-hydrolase activity Relationships: is a type of GO:0004553